metanephric S-shaped body morphogenesis [GO:0072284] (BP) Regulation: regulated by GO:2000004; negatively regulated by negative regulation of metanephric S-shaped body morphogenesis [GO:2000005] Definition: The process in which the metanephric S-shaped body is generated and organized. The metanephric S-shaped body is the successor of the metanephric comma-shaped body that contributes to the morphogenesis of a nephron in the metanephros. Relationships: is a type of S-shaped body morphogenesis [GO:0072050]; is part of GO:0072273 Sources: GOC:mtg_kidney_jan10